{
  "term_id": "GO:0007165",
  "gene_name": "Cyclin-dependent kinase 3",
  "term_label": "signal transduction",
  "gene": "UniProtKB:Q00526",
  "gene_symbol": "CDK3"
}